fungal-type vacuole membrane [GO:0000329] (cellular component) Definition: The lipid bilayer surrounding a vacuole, the shape of which correlates with cell cycle phase. The membrane separates its contents from the cytoplasm of the cell. An example of this structure is found in Saccharomyces cerevisiae. Sources: GOC:krc, GOC:mtg_sensu Also known as: membrane of vacuole with cell cycle-correlated morphology, fungal-type vacuolar membrane Relationships: is a type of lytic vacuole membrane [GO:0098852]; is part of fungal-type vacuole [GO:0000324]